{
  "gene": "UniProtKB:Q03113",
  "gene_name": "Guanine nucleotide-binding protein subunit alpha-12",
  "gene_symbol": "GNA12",
  "term_label": "cytoplasm",
  "term_id": "GO:0005737"
}